{
  "term_id": "GO:0000978",
  "gene_name": "Homeobox protein Hox-A4",
  "term_label": "RNA polymerase II cis-regulatory region sequence-specific DNA binding",
  "gene": "UniProtKB:Q00056",
  "gene_symbol": "HOXA4"
}